{
  "term_label": "sensory perception of sound",
  "gene_name": "Harmonin",
  "term_id": "GO:0007605",
  "gene_symbol": "USH1C",
  "gene": "UniProtKB:Q9Y6N9"
}